{
  "gene_name": "Tetratricopeptide repeat protein 29",
  "gene": "UniProtKB:Q8NA56",
  "term_label": "Unknown molecular function",
  "term_id": "UNKNOWN:0001",
  "gene_symbol": "TTC29"
}